negative regulation of 3'-UTR-mediated mRNA stabilization [GO:1905869] (biological process) Definition: Any process that stops, prevents or reduces the frequency, rate or extent of 3'-UTR-mediated mRNA stabilization. References: PMID:19737525 Sources: GOC:TermGenie, GO_REF:0000058 Relationships: is a type of GO:0048519; is_a positive regulation of mRNA catabolic process [GO:0061014]; is_a regulation of 3'-UTR-mediated mRNA stabilization [GO:1905868]; RO_0002212 GO:0070935 Also known as: down regulation of 3'-UTR-mediated mRNA stabilization, down regulation of 3'-untranslated region-mediated mRNA stabilization, down-regulation of 3'-UTR-mediated mRNA stabilization, down-regulation of 3'-untranslated region-mediated mRNA stabilization, downregulation of 3'-UTR-mediated mRNA stabilization, downregulation of 3'-untranslated region-mediated mRNA stabilization, negative regulation of 3'-untranslated region-mediated mRNA stabilization, inhibition of 3'-UTR-mediated mRNA stabilization, inhibition of 3'-untranslated region-mediated mRNA stabilization